{
  "term_id": "GO:0005886",
  "gene_symbol": "MPIG6B",
  "gene_name": "Megakaryocyte and platelet inhibitory receptor G6b",
  "gene": "UniProtKB:O95866",
  "term_label": "plasma membrane"
}